{
  "gene_symbol": "MAPK8IP2",
  "gene": "UniProtKB:Q13387",
  "gene_name": "C-Jun-amino-terminal kinase-interacting protein 2",
  "term_id": "GO:0005078",
  "term_label": "MAP-kinase scaffold activity"
}